{
  "gene_symbol": "TTC41P",
  "term_label": "Unknown cellular component",
  "term_id": "UNKNOWN:0003",
  "gene": "UniProtKB:Q6P2S7",
  "gene_name": "Putative tetratricopeptide repeat protein 41"
}